isovitexin beta-glucosyltransferase activity [GO:0050010] (molecular function) Relationships: is a type of GO:0035251 Definition: Catalysis of the reaction: isovitexin + UDP-D-glucose = H+ + isovitexin 2''-O-beta-D-glucoside + UDP. Also known as: isovitexin b-glucosyltransferase activity, UDP-glucose:isovitexin 2''-O-beta-D-glucosyltransferase activity, UDPglucose:isovitexin 2''-O-beta-D-glucosyltransferase activity, uridine diphosphoglucose-isovitexin 2''-glucosyltransferase activity Sources: EC:2.4.1.106, RHEA:19529